{
  "gene_name": "Protein AKNAD1",
  "gene": "UniProtKB:Q5T1N1",
  "term_id": "UNKNOWN:0002",
  "term_label": "Unknown biological process",
  "gene_symbol": "AKNAD1"
}